{
  "term_label": "fatty-acyl-CoA binding",
  "gene_name": "Sterol O-acyltransferase 1",
  "gene": "UniProtKB:P35610",
  "term_id": "GO:0000062",
  "gene_symbol": "SOAT1"
}